{
  "term_label": "N-acylsphingosine amidohydrolase activity",
  "gene_symbol": "ACER3",
  "gene": "UniProtKB:Q9NUN7",
  "term_id": "GO:0017040",
  "gene_name": "Alkaline ceramidase 3"
}